arabinan biosynthetic process [GO:0035884] (biological process) Definition: The chemical reactions and pathways resulting in the formation of arabinan, a polysaccharide composed of arabinose residues. Sources: GOC:rs, ISBN:0198506732 Relationships: is a type of GO:0000271; is_a arabinan metabolic process [GO:0031221]